colon smooth muscle contraction [GO:1990765] (biological process) Definition: A process in which force is generated within smooth muscle tissue, resulting in a change in muscle geometry of the large intestine, exclusive of the rectum. The colon is that part of the large intestine that connects the small intestine to the rectum. Regulation: regulated by regulation of colon smooth muscle contraction [GO:1904341]; RO_0002212 by negative regulation of colon smooth muscle contraction [GO:1904342]; positively regulated by positive regulation of colon smooth muscle contraction [GO:1904343] References: PMID:24170253 Relationships: is a type of GO:0006939; is part of intestine smooth muscle contraction [GO:0014827]